intestinal motility [GO:0120054] (BP) References: PMID:15890336 Sources: GOC:sl Relationships: is a type of digestive system process [GO:0022600] Definition: Contractions of the intestinal tract that include peristalsis (moving contents onward) and non-peristaltic movement (moving contents back and forth). Subtypes: small intestinal transit [GO:0120055], large intestinal transit [GO:0120056]